{
  "gene_symbol": "DBNDD2",
  "term_label": "Unknown molecular function",
  "gene_name": "Dysbindin domain-containing protein 2",
  "gene": "UniProtKB:Q9BQY9",
  "term_id": "UNKNOWN:0001"
}